regulation of embryonic pattern specification [GO:1902875] (biological process) Also known as: regulation of embryonic pattern biosynthesis, regulation of embryonic pattern formation, regulation of ventral/lateral system Subtypes: negative regulation of embryonic pattern specification [GO:1902876], positive regulation of embryonic pattern specification [GO:1902877] References: PMID:16872597 Sources: GOC:TermGenie, GOC:mr, GO_REF:0000058 Definition: Any process that modulates the frequency, rate or extent of embryonic pattern specification. Relationships: is_a regulation of multicellular organismal process [GO:0051239]; regulates GO:0009880